{
  "term_id": "GO:0007399",
  "gene_name": "Apical endosomal glycoprotein",
  "gene_symbol": "MAMDC4",
  "term_label": "nervous system development",
  "gene": "UniProtKB:Q6UXC1"
}